{
  "term_label": "3-beta-hydroxysteroid 3-dehydrogenase (NADP+) activity",
  "term_id": "GO:0000253",
  "gene_name": "3-keto-steroid reductase_17-beta-hydroxysteroid dehydrogenase 7",
  "gene_symbol": "HSD17B7",
  "gene": "UniProtKB:P56937"
}